{
  "gene_symbol": "PFKFB4",
  "term_id": "GO:0004331",
  "gene_name": "6-phosphofructo-2-kinase_fructose-2,6-bisphosphatase 4",
  "term_label": "fructose-2,6-bisphosphate 2-phosphatase activity",
  "gene": "UniProtKB:Q16877"
}